{
  "gene": "UniProtKB:Q5RIA9",
  "gene_symbol": "ZNG1E",
  "term_label": "zinc ion binding",
  "term_id": "GO:0008270",
  "gene_name": "Zinc-regulated GTPase metalloprotein activator 1E"
}